ferredoxin-nitrate reductase activity [GO:0047889] (molecular function) Relationships: is a type of GO:0008940; is a type of oxidoreductase activity, acting on other nitrogenous compounds as donors, iron-sulfur protein as acceptor [GO:0016664] Definition: Catalysis of the reaction: nitrite + 2 oxidized [2Fe-2S]-[ferredoxin] + H2O = nitrate + 2 reduced [2Fe-2S]-[ferredoxin] + 2 H+. Sources: RHEA:21828 Also known as: assimilatory nitrate reductase activity, assimilatory ferredoxin-nitrate reductase activity, nitrate (ferredoxin) reductase activity, nitrite:ferredoxin oxidoreductase activity